{
  "gene": "UniProtKB:P18510",
  "term_id": "GO:0006955",
  "gene_symbol": "IL1RN",
  "gene_name": "Interleukin-1 receptor antagonist protein",
  "term_label": "immune response"
}